{
  "gene_name": "Tumor necrosis factor receptor superfamily member 6",
  "gene_symbol": "FAS",
  "term_label": "external side of plasma membrane",
  "term_id": "GO:0009897",
  "gene": "UniProtKB:P25445"
}